{
  "term_label": "cytoplasm",
  "gene": "UniProtKB:Q9NVF9",
  "gene_symbol": "ETNK2",
  "gene_name": "Ethanolamine kinase 2",
  "term_id": "GO:0005737"
}